positive regulation of collateral sprouting in absence of injury [GO:0048697] (biological process) Relationships: is a type of GO:0048672; is a type of regulation of collateral sprouting in absence of injury [GO:0048696]; positively regulates collateral sprouting in absence of injury [GO:0048669] Also known as: up regulation of collateral sprouting in the absence of injury, up-regulation of collateral sprouting in the absence of injury, upregulation of collateral sprouting in the absence of injury, activation of collateral sprouting in the absence of injury, stimulation of collateral sprouting in the absence of injury Definition: Any process that activates or increases the frequency, rate or extent of collateral sprouting in the absence of injury. Sources: GOC:dgh, GOC:dph, GOC:jid, GOC:lm